regulation of establishment or maintenance of cell polarity regulating cell shape [GO:2000769] (biological process) Definition: Any process that modulates the frequency, rate or extent of establishment or maintenance of cell polarity regulating cell shape. Sources: GOC:mah Relationships: is a type of regulation of cell shape [GO:0008360]; is a type of regulation of establishment or maintenance of cell polarity [GO:0032878]; regulates GO:0071963 Subtypes: GO:2000100, negative regulation of establishment or maintenance of cell polarity regulating cell shape [GO:2000770], positive regulation of establishment or maintenance of cell polarity regulating cell shape [GO:2000771], regulation of establishment of cell polarity regulating cell shape [GO:2000782]